{
  "term_id": "GO:0006868",
  "gene_name": "Sodium-coupled neutral amino acid symporter 2",
  "term_label": "glutamine transport",
  "gene": "UniProtKB:Q96QD8",
  "gene_symbol": "SLC38A2"
}